{
  "gene_name": "Arylacetamide deacetylase-like 3",
  "gene_symbol": "AADACL3",
  "term_id": "UNKNOWN:0003",
  "gene": "UniProtKB:Q5VUY0",
  "term_label": "Unknown cellular component"
}